neuron development [GO:0048666] (BP) Subtypes: pancreatic D cell development [GO:0003324], noradrenergic neuron development [GO:0003358], GO:0003388, GO:0021954, neuromast hair cell development [GO:0035675], GO:0042461, GO:0048935, inner ear receptor cell development [GO:0060119] Definition: The process whose specific outcome is the progression of a neuron over time, from initial commitment of the cell to a specific fate, to the fully functional differentiated cell. Relationships: is a type of cell development [GO:0048468]; is part of neuron differentiation [GO:0030182] Sources: GOC:dph